regulation of skeletal muscle cell differentiation [GO:2001014] (biological process) Subtypes: regulation of skeletal muscle fiber differentiation [GO:1902809], negative regulation of skeletal muscle cell differentiation [GO:2001015], positive regulation of skeletal muscle cell differentiation [GO:2001016] Relationships: is_a regulation of cell differentiation [GO:0045595]; regulates GO:0035914 Sources: GOC:obol Definition: Any process that modulates the frequency, rate or extent of skeletal muscle cell differentiation.